{
  "gene_symbol": "BTAF1",
  "gene": "UniProtKB:O14981",
  "gene_name": "TATA-binding protein-associated factor 172",
  "term_id": "UNKNOWN:0003",
  "term_label": "Unknown cellular component"
}